{
  "term_label": "early endosome to late endosome transport",
  "term_id": "GO:0045022",
  "gene_name": "Rab-interacting lysosomal protein",
  "gene_symbol": "RILP",
  "gene": "UniProtKB:Q96NA2"
}